calcium:monoatomic cation antiporter activity involved in regulation of presynaptic cytosolic calcium ion concentration [GO:1905055] (molecular function) References: PMID:22972962, PMID:23255722 Sources: GOC:TermGenie, GO_REF:0000061 Relationships: is a type of GO:0015368; BFO_0000050 regulation of presynaptic cytosolic calcium ion concentration [GO:0099509] Also known as: calcium:cation antiporter activity involved in regulation of presynaptic cytosolic calcium ion concentration, calcium ion antiporter activity involved in regulation of presynaptic cytosolic calcium levels Definition: Any calcium:cation antiporter activity that is involved in regulation of presynaptic cytosolic calcium ion concentration.